{
  "gene_symbol": "USP2",
  "term_label": "Unknown molecular function",
  "term_id": "UNKNOWN:0001",
  "gene": "UniProtKB:O75604",
  "gene_name": "Ubiquitin carboxyl-terminal hydrolase 2"
}